presynaptic active zone dense projection [GO:0097445] (CC) Definition: Electron dense projection extending from the cytomatrix into the cytoplasm on which synaptic vesicles are tethered. Also known as: active zone dense projection, pre-synaptic active zone dense projection Relationships: is a type of cellular anatomical structure [GO:0110165]; is part of presynaptic active zone [GO:0048786] References: PMID:15381754 Sources: NIF_Subcellular:sao494258938